Golgi-associated vesicle membrane [GO:0030660] (cellular component) Definition: The lipid bilayer surrounding a vesicle associated with the Golgi apparatus. Sources: GOC:mah Also known as: Golgi vesicle membrane Relationships: is a type of cytoplasmic vesicle membrane [GO:0030659]; is a type of bounding membrane of organelle [GO:0098588]; is part of Golgi-associated vesicle [GO:0005798] Subtypes: trans-Golgi network transport vesicle membrane [GO:0012510], COPI-coated vesicle membrane [GO:0030663]